{
  "gene": "UniProtKB:P13861",
  "term_label": "cytosol",
  "gene_symbol": "PRKAR2A",
  "term_id": "GO:0005829",
  "gene_name": "cAMP-dependent protein kinase type II-alpha regulatory subunit"
}